{
  "term_id": "GO:0001649",
  "gene_symbol": "MYOC",
  "gene": "UniProtKB:Q99972",
  "gene_name": "Myocilin",
  "term_label": "osteoblast differentiation"
}